{
  "term_id": "GO:0003924",
  "gene": "UniProtKB:P61587",
  "gene_name": "Rho-related GTP-binding protein RhoE",
  "term_label": "GTPase activity",
  "gene_symbol": "RND3"
}